{
  "gene": "UniProtKB:Q6ZV73",
  "gene_name": "FYVE, RhoGEF and PH domain-containing protein 6",
  "term_id": "GO:0005737",
  "gene_symbol": "FGD6",
  "term_label": "cytoplasm"
}